{
  "gene_symbol": "FAM9A",
  "gene_name": "Protein FAM9A",
  "gene": "UniProtKB:Q8IZU1",
  "term_label": "Unknown molecular function",
  "term_id": "UNKNOWN:0001"
}